Parkin-FBXW7-Cul1 ubiquitin ligase complex [GO:1990452] (cellular component) Also known as: PRKN-FBXW7-Cul1 complex, Park2-FBXW7-Cul1 complex, Parkin-FBXW7-Cul1 protein complex, Parkin/Cul1/F-box protein complex, Parkin-HSel-10-Cullin-1 complex References: PMID:12628165 Sources: GOC:PARL, GOC:bf Relationships: is a type of ubiquitin ligase complex [GO:0000151] Definition: A ubiquitin ligase complex containing Parkin (PARK2), the F-box protein FBXW7 (also called SEL-10) and a cullin from the Cul1 subfamily; substrate specificity is conferred by the F-box protein.